{
  "gene_name": "Mitochondrial import inner membrane translocase subunit Tim17-B",
  "term_id": "GO:0005744",
  "gene": "UniProtKB:O60830",
  "term_label": "TIM23 mitochondrial import inner membrane translocase complex",
  "gene_symbol": "TIMM17B"
}